regulation of neuronal synaptic plasticity in response to neurotrophin [GO:0031637] (biological process) References: PMID:8703078 Sources: GOC:mah Relationships: is a type of GO:0048168 Definition: The process in which a neurotrophic factor induces neuronal synaptic plasticity, the ability of neuronal synapses to change as circumstances require. They may alter function, such as increasing or decreasing their sensitivity, or they may increase or decrease in actual numbers. Also known as: neurotrophin-induced neuronal synaptic plasticity